{
  "gene_symbol": "MAP7D1",
  "term_id": "UNKNOWN:0001",
  "gene": "UniProtKB:Q3KQU3",
  "gene_name": "MAP7 domain-containing protein 1",
  "term_label": "Unknown molecular function"
}